leaf proximal/distal pattern formation [GO:0010589] (biological process) Definition: The regionalization process within a leaf by which specific areas of cell differentiation are determined along a proximal/distal axis. References: PMID:18398054 Relationships: is a type of GO:0009954